{
  "gene_name": "Phosphatidate cytidylyltransferase, mitochondrial",
  "term_id": "GO:0032049",
  "term_label": "cardiolipin biosynthetic process",
  "gene_symbol": "TAMM41",
  "gene": "UniProtKB:Q96BW9"
}